glutamate receptor clustering [GO:0097688] (biological process) Relationships: is a type of neurotransmitter-gated ion channel clustering [GO:0072578] Definition: The neurotransmitter-gated ion channel clustering process in which glutamate receptors are localized to distinct domains in the cell membrane. Also known as: glutamatergic receptor clustering Subtypes: GO:0097113 References: PMID:19723286 Sources: GOC:krc Regulation: RO_0002211 by GO:0106104